meiotic DNA repair synthesis involved in meiotic gene conversion [GO:0010779] (biological process) Sources: GOC:dph, GOC:tb Relationships: is a type of meiotic DNA repair synthesis [GO:0000711]; is part of meiotic gene conversion [GO:0006311] Definition: The synthesis of DNA proceeding from the broken 3' single-strand DNA end that uses the homologous intact duplex as the template resulting in meiotic gene conversion. Meiotic gene conversion is the cell cycle process in which genetic information is transferred from one helix to another.